{
  "term_label": "Unknown biological process",
  "gene": "UniProtKB:A0A075B6Z8",
  "gene_symbol": "TRAJ25",
  "gene_name": "T cell receptor alpha joining 25 (non-functional) (Fragment)",
  "term_id": "UNKNOWN:0002"
}